{
  "term_label": "Unknown biological process",
  "gene_symbol": "A8MX80",
  "gene": "UniProtKB:A8MX80",
  "term_id": "UNKNOWN:0002",
  "gene_name": "Putative UPF0607 protein ENSP00000383144"
}